{
  "gene_name": "Small nuclear ribonucleoprotein Sm D3",
  "gene": "UniProtKB:P62318",
  "term_label": "U2 snRNP",
  "gene_symbol": "SNRPD3",
  "term_id": "GO:0005686"
}